{
  "term_label": "keratin filament",
  "term_id": "GO:0045095",
  "gene_symbol": "KRT1",
  "gene_name": "Keratin, type II cytoskeletal 1",
  "gene": "UniProtKB:P04264"
}